{
  "gene_symbol": "CES3",
  "gene": "UniProtKB:Q6UWW8",
  "term_label": "Unknown cellular component",
  "gene_name": "Carboxylesterase 3",
  "term_id": "UNKNOWN:0003"
}